{
  "gene_name": "Sterile alpha motif domain-containing protein 14",
  "term_label": "cytoplasm",
  "term_id": "GO:0005737",
  "gene_symbol": "SAMD14",
  "gene": "UniProtKB:Q8IZD0"
}